L-lysine N-acetyltransferase activity, acting on acetyl phosphate as donor [GO:0004468] (molecular function) Also known as: lysine N-acetyltransferase activity, acting on acetyl phosphate as donor, lysine acetyltransferase activity, LAT activity, acetyl-phosphate:L-lysine 6-N-acetyltransferase activity, acetyl-phosphate:L-lysine N6-acetyltransferase activity, lysine N(6)-acetyltransferase activity, lysine N6-acetyltransferase activity Relationships: is a type of L-amino-acid N-acetyltransferase activity [GO:0140085] Definition: Catalysis of the reaction: acetyl phosphate + L-lysine = phosphate + N6-acetyl-L-lysine. Sources: RHEA:14417